{
  "gene": "UniProtKB:Q07001",
  "term_label": "acetylcholine-gated channel complex",
  "gene_symbol": "CHRND",
  "term_id": "GO:0005892",
  "gene_name": "Acetylcholine receptor subunit delta"
}